{
  "term_label": "glycoprotein biosynthetic process",
  "term_id": "GO:0009101",
  "gene_name": "Galactose-3-O-sulfotransferase 2",
  "gene_symbol": "GAL3ST2",
  "gene": "UniProtKB:Q9H3Q3"
}